{
  "gene_symbol": "IFNE",
  "term_label": "adaptive immune response",
  "gene": "UniProtKB:Q86WN2",
  "gene_name": "Interferon epsilon",
  "term_id": "GO:0002250"
}